{
  "gene_name": "Ras-related protein Rab-35",
  "gene_symbol": "RAB35",
  "gene": "UniProtKB:Q15286",
  "term_id": "GO:0032456",
  "term_label": "endocytic recycling"
}